disaccharide biosynthetic process [GO:0046351] (biological process) Subtypes: maltose biosynthetic process [GO:0000024], GO:0005986, lactose biosynthetic process [GO:0005989], trehalose biosynthetic process [GO:0005992], melibiose biosynthetic process [GO:0042544] Sources: GOC:ai Also known as: disaccharide anabolism, disaccharide biosynthesis, disaccharide formation, disaccharide synthesis Definition: The chemical reactions and pathways resulting in the formation of disaccharides, sugars composed of two monosaccharide units. Relationships: is a type of disaccharide metabolic process [GO:0005984]; is a type of oligosaccharide biosynthetic process [GO:0009312]